positive regulation of complement activation, lectin pathway [GO:0001870] (BP) Definition: Any process that activates or increases the frequency, rate or extent of complement activation by the lectin pathway. Also known as: positive regulation of complement cascade, lectin pathway, up regulation of complement activation, lectin pathway, up-regulation of complement activation, lectin pathway, upregulation of complement activation, lectin pathway, activation of complement activation, lectin pathway, stimulation of complement activation, lectin pathway Relationships: is a type of regulation of complement activation, lectin pathway [GO:0001868]; is a type of positive regulation of innate immune response [GO:0045089]; is a type of positive regulation of complement activation [GO:0045917]; positively regulates complement activation, lectin pathway [GO:0001867] Sources: GOC:add, ISBN:0781735149